{
  "gene": "UniProtKB:Q5VWM3",
  "term_id": "GO:0031462",
  "term_label": "Cul2-RING ubiquitin ligase complex",
  "gene_symbol": "PRAMEF18",
  "gene_name": "PRAME family member 18"
}